{
  "gene_symbol": "NFKB1",
  "gene_name": "Nuclear factor NF-kappa-B p105 subunit",
  "gene": "UniProtKB:P19838",
  "term_label": "NF-kappaB p50/p65 complex",
  "term_id": "GO:0035525"
}